cellular response to ether [GO:0071362] (biological process) Subtypes: cellular response to trichodermin [GO:0072744], cellular response to rapamycin [GO:0072752], cellular response to differentiation-inducing factor 1 [GO:1903014], cellular response to 2-O-acetyl-1-O-hexadecyl-sn-glycero-3-phosphocholine [GO:1904317], cellular response to dextromethorphan [GO:1904559], cellular response to ionomycin [GO:1904637], cellular response to curcumin [GO:1904644] Sources: GOC:mah Relationships: is a type of response to ether [GO:0045472]; is_a cellular response to oxygen-containing compound [GO:1901701] Definition: Any process that results in a change in state or activity of a cell (in terms of movement, secretion, enzyme production, gene expression, etc.) as a result of a ether stimulus.